{
  "gene": "UniProtKB:Q9UK33",
  "gene_symbol": "ZNF580",
  "gene_name": "Zinc finger protein 580",
  "term_id": "GO:0005634",
  "term_label": "nucleus"
}